biopterin transmembrane transporter activity [GO:0015224] (molecular function) Also known as: biopterin transporter activity Definition: Enables the transfer of biopterin from one side of a membrane to the other. Biopterin is a growth factor for certain protozoans and some insects; it is widely distributed in tissues and functions in a reduced form, tetrahydrobiopterin, as a hydroxylation coenzyme. Relationships: is a type of GO:0022857; is part of biopterin transport [GO:0015877] Sources: ISBN:0198506732